{
  "gene": "UniProtKB:Q16526",
  "gene_symbol": "CRY1",
  "term_label": "nucleus",
  "term_id": "GO:0005634",
  "gene_name": "Cryptochrome-1"
}